{
  "gene_name": "Membrane protein MLC1",
  "gene_symbol": "MLC1",
  "term_id": "GO:0005783",
  "gene": "UniProtKB:Q15049",
  "term_label": "endoplasmic reticulum"
}